{
  "term_label": "G protein-coupled receptor activity",
  "gene": "UniProtKB:Q14246",
  "term_id": "GO:0004930",
  "gene_symbol": "ADGRE1",
  "gene_name": "Adhesion G protein-coupled receptor E1"
}